{
  "gene": "UniProtKB:Q8N1F7",
  "term_id": "GO:0017056",
  "gene_symbol": "NUP93",
  "term_label": "structural constituent of nuclear pore",
  "gene_name": "Nuclear pore complex protein Nup93"
}